{
  "term_label": "immune response-inhibiting cell surface receptor signaling pathway",
  "gene_name": "Leukocyte immunoglobulin-like receptor subfamily A member 1",
  "term_id": "GO:0002767",
  "gene": "UniProtKB:O75019",
  "gene_symbol": "LILRA1"
}